{
  "gene_symbol": "ALDH16A1",
  "gene_name": "Aldehyde dehydrogenase family 16 member A1",
  "term_label": "aldehyde dehydrogenase (NAD+) activity",
  "gene": "UniProtKB:Q8IZ83",
  "term_id": "GO:0004029"
}